regulation of regulated secretory pathway [GO:1903305] (biological process) References: PMID:12526776 Sources: GOC:PARL, GOC:TermGenie, GOC:pad, GO_REF:0000058 Relationships: is a type of regulation of exocytosis [GO:0017157]; regulates regulated exocytosis [GO:0045055] Definition: Any process that modulates the frequency, rate or extent of regulated secretory pathway. Note: An example of this is protein domain-specific expression of Synaptotagmin 1 in rat (P21707) in PMID:12526776 inferred from mutant phenotype. Subtypes: GO:0017158, regulation of leukocyte degranulation [GO:0043300], negative regulation of regulated secretory pathway [GO:1903306], positive regulation of regulated secretory pathway [GO:1903307], regulation of synaptic vesicle exocytosis [GO:2000300]